{
  "gene_name": "Delta(14)-sterol reductase LBR",
  "gene": "UniProtKB:Q14739",
  "term_label": "Delta14-sterol reductase activity",
  "term_id": "GO:0050613",
  "gene_symbol": "LBR"
}